{
  "gene_name": "Calcium_calmodulin-dependent protein kinase type II subunit alpha",
  "gene": "UniProtKB:Q9UQM7",
  "term_id": "GO:0048168",
  "term_label": "regulation of neuronal synaptic plasticity",
  "gene_symbol": "CAMK2A"
}